{
  "term_id": "GO:0005763",
  "gene_symbol": "MRPS18C",
  "term_label": "mitochondrial small ribosomal subunit",
  "gene_name": "Small ribosomal subunit protein bS18m",
  "gene": "UniProtKB:Q9Y3D5"
}